{
  "gene_symbol": "KCNJ18",
  "gene": "UniProtKB:B7U540",
  "term_label": "potassium ion import across plasma membrane",
  "term_id": "GO:1990573",
  "gene_name": "Inward rectifier potassium channel 18"
}